regulation of NADP metabolic process [GO:1902031] (BP) Also known as: regulation of NADP (oxidized) metabolic process, regulation of NADP (oxidized) metabolism, regulation of NADP (reduced) metabolic process, regulation of NADP (reduced) metabolism, regulation of NADP metabolism, regulation of NADPH metabolic process, regulation of NADPH metabolism, regulation of nicotinamide adenine dinucleotide phosphate metabolic process, regulation of nicotinamide adenine dinucleotide phosphate metabolism, regulation of oxidized NADP metabolic process, regulation of oxidized NADP metabolism, regulation of oxidized nicotinamide adenine dinucleotide phosphate metabolic process, regulation of oxidized nicotinamide adenine dinucleotide phosphate metabolism, regulation of reduced NADP metabolic process, regulation of reduced NADP metabolism, regulation of reduced nicotinamide adenine dinucleotide phosphate metabolic process, regulation of reduced nicotinamide adenine dinucleotide phosphate metabolism, regulation of NAD phosphorylation and dephosphorylation Subtypes: regulation of pentose-phosphate shunt [GO:0043456] References: PMID:23334421 Sources: GOC:TermGenie Definition: Any process that modulates the frequency, rate or extent of NADP metabolic process. Relationships: is_a GO:1900542; regulates NADP+ metabolic process [GO:0006739]